neuromast deposition [GO:0048885] (BP) References: PMID:15018940 Subtypes: anterior lateral line neuromast deposition [GO:0048902], posterior lateral line neuromast deposition [GO:0048922] Relationships: is a type of negative regulation of cell migration [GO:0030336]; is part of GO:0048884 Definition: The process in which a migrating neuromast primordium deposits clusters of undifferentiated cells (proneuromasts) along its migratory path in a developing lateral line.